norsolorinate anthrone synthase activity [GO:0102973] (molecular function) Sources: EC:2.3.1.221, GOC:pz Relationships: is a type of GO:0016747 Also known as: norsolorinic acid synthase Definition: Catalysis of the reaction: 7 malonyl-CoA + 5 H+ + a hexanoyl-[acyl-carrier-protein] = norsolorinate anthrone + 7 coenzyme A + 7 carbon dioxide + 2 H2O + a holo-[acyl-carrier protein].